regulation of transcription by galactose [GO:0000409] (biological process) Subtypes: GO:0000410, positive regulation of transcription by galactose [GO:0000411], regulation of transcription from RNA polymerase II promoter by galactose [GO:0000431] Sources: GOC:go_curators Definition: Any process involving galactose that modulates the frequency, rate or extent or transcription. Relationships: is a type of regulation of DNA-templated transcription [GO:0006355]